{
  "term_label": "Unknown biological process",
  "term_id": "UNKNOWN:0002",
  "gene_name": "Nuclear apoptosis-inducing factor 1",
  "gene": "UniProtKB:Q69YI7",
  "gene_symbol": "NAIF1"
}